{
  "gene": "UniProtKB:P29376",
  "gene_name": "Leukocyte tyrosine kinase receptor",
  "gene_symbol": "LTK",
  "term_label": "regulation of cell population proliferation",
  "term_id": "GO:0042127"
}